CDP reductase activity [GO:0051063] (molecular function) Definition: Catalysis of the reaction: dCDP + thioredoxin disulfide + H2O = CDP + thioredoxin. Also known as: CDP reduction Sources: MetaCyc:CDPREDUCT-RXN Relationships: is a type of GO:0004748